{
  "term_label": "DNA-binding transcription factor activity, RNA polymerase II-specific",
  "term_id": "GO:0000981",
  "gene": "UniProtKB:O15119",
  "gene_symbol": "TBX3",
  "gene_name": "T-box transcription factor TBX3"
}